{
  "gene_name": "Immediate early response gene 5 protein",
  "term_id": "UNKNOWN:0003",
  "term_label": "Unknown cellular component",
  "gene_symbol": "IER5",
  "gene": "UniProtKB:Q5VY09"
}